negative regulation of androgen receptor signaling pathway [GO:0060766] (biological process) Also known as: negative regulation of androgen receptor signalling pathway Relationships: is a type of negative regulation of intracellular steroid hormone receptor signaling pathway [GO:0033144]; is a type of regulation of androgen receptor signaling pathway [GO:0060765]; negatively regulates androgen receptor signaling pathway [GO:0030521] Sources: GOC:dph Definition: Any process that decreases the rate, frequency, or extent of the androgen receptor signaling pathway.